{
  "gene": "UniProtKB:Q8N9U0",
  "gene_name": "Tandem C2 domains nuclear protein",
  "term_label": "Unknown biological process",
  "term_id": "UNKNOWN:0002",
  "gene_symbol": "TC2N"
}